venom-mediated activation of G protein-coupled receptor signaling pathway [GO:0044514] (biological process) Subtypes: GO:0140183 Definition: A process in which an organism initiates, promotes, or enhances a G protein-coupled receptor signaling pathway in another organism via the action of a venom. Relationships: is a type of venom-mediated perturbation of G protein-coupled receptor signaling pathway [GO:0044513] References: PMID:8405712 Sources: GOC:fj, GOC:jl Also known as: envenomation resulting in positive regulation of G protein-coupled receptor activity in another organism, envenomation resulting in positive regulation of G protein-coupled receptor activity in other organism, envenomation resulting in positive regulation of G-protein coupled receptor activity in other organism